{
  "gene_name": "Centriole and centriolar satellite protein OFD1",
  "term_label": "centrosome",
  "term_id": "GO:0005813",
  "gene_symbol": "OFD1",
  "gene": "UniProtKB:O75665"
}